granulocyte macrophage colony-stimulating factor production [GO:0032604] (biological process) Also known as: GM-CSF production, granulocyte macrophage colony stimulating factor production, granulocyte macrophage colony-stimulating factor biosynthetic process Relationships: is a type of cytokine production [GO:0001816]; is a type of protein metabolic process [GO:0019538] Sources: GOC:mah, ISBN:0198506732 Regulation: regulated by GO:0032645; negatively regulated by negative regulation of granulocyte macrophage colony-stimulating factor production [GO:0032685]; positively regulated by GO:0032725 Definition: The appearance of granulocyte macrophage colony-stimulating factor due to biosynthesis or secretion following a cellular stimulus, resulting in an increase in its intracellular or extracellular levels.